{
  "gene": "UniProtKB:Q59H18",
  "gene_symbol": "TNNI3K",
  "term_label": "regulation of cardiac muscle contraction",
  "gene_name": "Serine_threonine-protein kinase TNNI3K",
  "term_id": "GO:0055117"
}